{
  "gene_symbol": "STRC",
  "term_label": "Unknown molecular function",
  "term_id": "UNKNOWN:0001",
  "gene": "UniProtKB:Q7RTU9",
  "gene_name": "Stereocilin"
}